negative regulation of dendrite morphogenesis [GO:0050774] (biological process) Also known as: down regulation of dendrite morphogenesis, down-regulation of dendrite morphogenesis, downregulation of dendrite morphogenesis, inhibition of dendrite morphogenesis Sources: GOC:ai Definition: Any process that stops, prevents, or reduces the frequency, rate or extent of dendrite morphogenesis. Relationships: is a type of negative regulation of cell projection organization [GO:0031345]; is a type of GO:0048814; is a type of negative regulation of neurogenesis [GO:0050768]; negatively regulates GO:0048813